{
  "gene_name": "Arginase-1",
  "gene": "UniProtKB:P05089",
  "term_id": "GO:0004053",
  "term_label": "arginase activity",
  "gene_symbol": "ARG1"
}